pyrimidine nucleobase binding [GO:0002061] (molecular function) Also known as: pyrimidine base binding, 1,3-diazine binding, pyrimidine binding Relationships: is_a nucleobase binding [GO:0002054] Definition: Binding to a pyrimidine nucleobase, an organic nitrogenous base with a pyrimidine skeleton. Subtypes: cytosine binding [GO:0002056], uracil binding [GO:0002058], thymine binding [GO:0002059] Sources: GOC:hjd